{
  "gene_name": "Putative pro-MCH-like protein 1",
  "term_label": "type 1 melanin-concentrating hormone receptor binding",
  "gene": "UniProtKB:Q16048",
  "gene_symbol": "PMCHL1",
  "term_id": "GO:0031777"
}